{
  "term_label": "Unknown biological process",
  "gene_symbol": "EMC1",
  "term_id": "UNKNOWN:0002",
  "gene": "UniProtKB:Q8N766",
  "gene_name": "ER membrane protein complex subunit 1"
}